{
  "gene_symbol": "LGALS3",
  "term_id": "GO:0002548",
  "gene_name": "Galectin-3",
  "term_label": "monocyte chemotaxis",
  "gene": "UniProtKB:P17931"
}